{
  "gene_name": "Zinc finger protein 438",
  "term_id": "GO:0005634",
  "term_label": "nucleus",
  "gene_symbol": "ZNF438",
  "gene": "UniProtKB:Q7Z4V0"
}